{
  "gene_symbol": "IGHV3-72",
  "term_label": "immunoglobulin mediated immune response",
  "term_id": "GO:0016064",
  "gene_name": "Immunoglobulin heavy variable 3-72",
  "gene": "UniProtKB:A0A0B4J1Y9"
}